hepatic stellate cell activation [GO:0035733] (biological process) Sources: CL:0000632, GOC:bf Definition: A change in the morphology or behavior of a hepatic stellate cell resulting from exposure to a cytokine, chemokine, hormone, cellular ligand or soluble factor. Relationships: is a type of fibroblast activation [GO:0072537] Regulation: regulated by GO:2000489; negatively regulated by negative regulation of hepatic stellate cell activation [GO:2000490]; positively regulated by positive regulation of hepatic stellate cell activation [GO:2000491]